methylglyoxal biosynthetic process [GO:0019242] (biological process) Also known as: methylglyoxal anabolism, methylglyoxal biosynthesis, methylglyoxal formation, methylglyoxal synthesis Definition: The chemical reactions and pathways resulting in the formation of methylglyoxal, CH3-CO-CHO, the aldehyde of pyruvic acid. Sources: GOC:ai Relationships: is a type of GO:0009438; is a type of ketone biosynthetic process [GO:0042181]; is a type of aldehyde biosynthetic process [GO:0046184]